phosphoadenylyl-sulfate reductase (thioredoxin) activity [GO:0004604] (molecular function) Relationships: is a type of oxidoreductase activity, acting on a sulfur group of donors, disulfide as acceptor [GO:0016671] Also known as: phosphoadenylyl-sulphate reductase (thioredoxin) activity, 3'-phosphoadenylylsulfate reductase activity, PAPS reductase activity, PAPS reductase, thioredoxin-dependent activity, PAPS sulfotransferase activity, PAdoPS reductase activity, adenosine 3',5'-bisphosphate,sulfite:oxidized-thioredoxin oxidoreductase (3'-phosphoadenosine-5'-phosphosulfate-forming), adenosine 3',5'-bisphosphate,sulfite:thioredoxin-disulfide oxidoreductase (3'-phosphoadenosine-5'-phosphosulfate-forming), phosphoadenosine-phosphosulfate reductase activity, thioredoxin:3'-phospho-adenylylsulfate reductase activity, thioredoxin:adenosine 3'-phosphate 5'-phosphosulfate reductase activity Definition: Catalysis of the reaction: adenosine 3',5'-diphosphate + H+ + sulfite + thioredoxin disulfide = 3'-phospho-5'-adenylyl sulfate + thioredoxin. Thioredoxin disulfide is the oxidized form of thioredoxin; 3'-phosphoadenosine 5'-phosphosulfate is also known as PAPS. Sources: EC:1.8.4.8, RHEA:11724